actin filament bundle convergence [GO:0090426] (biological process) Relationships: is a type of GO:0070650 Subtypes: GO:0071520 Definition: A process of actin filament bundle distribution that results in the compaction of actin filaments. Sources: GOC:dph, GOC:tb